{
  "gene_name": "Protein TANC1",
  "gene": "UniProtKB:Q9C0D5",
  "term_label": "regulation of postsynapse organization",
  "gene_symbol": "TANC1",
  "term_id": "GO:0099175"
}